{
  "gene_symbol": "MMP25",
  "term_id": "GO:0005615",
  "gene": "UniProtKB:Q9NPA2",
  "gene_name": "Matrix metalloproteinase-25",
  "term_label": "extracellular space"
}